{
  "gene": "UniProtKB:Q9Y2R2",
  "term_label": "T cell receptor signaling pathway",
  "gene_name": "Tyrosine-protein phosphatase non-receptor type 22",
  "gene_symbol": "PTPN22",
  "term_id": "GO:0050852"
}